RNA polymerase II general transcription initiation factor binding [GO:0001091] (molecular function) Definition: Binding to a basal RNA polymerase II transcription factor, any of the factors involved in formation of the preinitiation complex (PIC) by RNA polymerase II and defined as a basal or general transcription factor. Relationships: is a type of basal RNA polymerase II transcription machinery binding [GO:0001099]; is a type of general transcription initiation factor binding [GO:0140296] Subtypes: TFIIA-class transcription factor complex binding [GO:0001092], GO:0001093, TFIID-class transcription factor complex binding [GO:0001094], TFIIE-class transcription factor complex binding [GO:0001095], TFIIF-class transcription factor complex binding [GO:0001096], TFIIH-class transcription factor complex binding [GO:0001097] Also known as: RNA polymerase II basal transcription factor binding References: PMID:16858867 Sources: GOC:txnOH